{
  "term_label": "guanyl-nucleotide exchange factor activity",
  "gene": "UniProtKB:Q9HD47",
  "gene_symbol": "RANGRF",
  "gene_name": "Ran guanine nucleotide release factor",
  "term_id": "GO:0005085"
}